{
  "gene_name": "Long-chain fatty acid transport protein 5",
  "term_id": "GO:0001676",
  "term_label": "long-chain fatty acid metabolic process",
  "gene": "UniProtKB:Q9Y2P5",
  "gene_symbol": "SLC27A5"
}